{
  "gene_symbol": "CDH23",
  "term_id": "GO:0031175",
  "term_label": "neuron projection development",
  "gene_name": "Cadherin-23",
  "gene": "UniProtKB:Q9H251"
}